caffeine oxidase activity [GO:0034875] (molecular function) Definition: Catalysis of the reaction: caffeine + O2 + 2 H+ + 2 e- = 1,3,7-trimethyluric acid + H2O. Relationships: is a type of GO:0033695 Sources: RHEA:47148